regulation of oomycete sporangium development [GO:0075322] (biological process) Definition: Any process that modulates the frequency, rate or extent of oomycete sporangium development, a process that leads to the formation of oomycete sporangium, a single-celled or many-celled structure that germinates directly to form an infection hypha or differentiate, through specialized cleavage vesicles, into between 10 and 30 zoospores, which is laterally flagellated. Relationships: is_a regulation of asexual sporulation [GO:0034305]; is a type of GO:0075310; regulates oomycete sporangium development [GO:0075321] Subtypes: positive regulation of oomycete sporangium development [GO:0075323], negative regulation of oomycete sporangium development [GO:0075324] Sources: GOC:pamgo_curators